{
  "term_id": "GO:0120162",
  "gene_symbol": "UCP2",
  "gene_name": "Dicarboxylate carrier SLC25A8",
  "gene": "UniProtKB:P55851",
  "term_label": "positive regulation of cold-induced thermogenesis"
}